{
  "gene": "UniProtKB:Q9ULD4",
  "term_id": "GO:0006338",
  "gene_name": "Bromodomain and PHD finger-containing protein 3",
  "term_label": "chromatin remodeling",
  "gene_symbol": "BRPF3"
}